{
  "gene_symbol": "OR51C1",
  "gene_name": "Olfactory receptor",
  "term_label": "Unknown biological process",
  "term_id": "UNKNOWN:0002",
  "gene": "UniProtKB:A0A3B3IT45"
}